{
  "gene_symbol": "GINS3",
  "term_label": "GINS complex",
  "gene": "UniProtKB:Q9BRX5",
  "term_id": "GO:0000811",
  "gene_name": "DNA replication complex GINS protein PSF3"
}